antigen processing and presentation following pinocytosis [GO:0002746] (biological process) Relationships: is_a antigen processing and presentation [GO:0019882] Subtypes: GO:0002421, antigen processing and presentation following macropinocytosis [GO:0002750] Definition: Antigen processing and presentation which is initiated by uptake of antigen via pinocytosis. Sources: GOC:add, ISBN:0781735149